AF-1 domain binding [GO:0050683] (molecular function) Definition: Binding to an AF-1 protein domain, a ligand-independent transactivation domain which is required for the full transcriptional activity of the receptor. Relationships: is a type of protein domain specific binding [GO:0019904] References: PMID:9682036